asparaginyl-tRNA synthase (glutamine-hydrolyzing) activity [GO:0050566] (molecular function) Definition: Catalysis of the reaction: L-glutamine + aspartyl-tRNA(Asn) + ATP = L-glutamate + asparaginyl-tRNA(Asn) + phosphate + ADP. Also known as: Asp-AdT activity, Asp-tRNA(Asn) amidotransferase activity, Asp-tRNAAsn amidotransferase activity, Asp-tRNAAsn:L-glutamine amido-ligase (ADP-forming), asparaginyl-tRNA synthase (glutamine-hydrolysing), aspartyl-tRNA(Asn) amidotransferase activity, aspartyl-tRNAAsn amidotransferase activity, aspartyl-tRNAAsn:L-glutamine amido-ligase (ADP-forming) Sources: EC:6.3.5.6, MetaCyc:6.3.5.6-RXN Relationships: is a type of carbon-nitrogen ligase activity, with glutamine as amido-N-donor [GO:0016884]; is a type of catalytic activity, acting on a tRNA [GO:0140101]